{
  "term_label": "positive regulation of phosphatidylinositol 3-kinase/protein kinase B signal transduction",
  "term_id": "GO:0051897",
  "gene_symbol": "IGF2",
  "gene": "UniProtKB:P01344",
  "gene_name": "Insulin-like growth factor II"
}